{
  "gene_symbol": "TRAV16",
  "term_id": "GO:0002250",
  "term_label": "adaptive immune response",
  "gene": "UniProtKB:A0A0A6YYK6",
  "gene_name": "T cell receptor alpha variable 16"
}